{
  "gene": "UniProtKB:O15342",
  "term_id": "UNKNOWN:0001",
  "gene_name": "V-type proton ATPase subunit e 1",
  "term_label": "Unknown molecular function",
  "gene_symbol": "ATP6V0E1"
}